{
  "term_label": "Unknown cellular component",
  "gene_symbol": "NPTX1",
  "gene_name": "Neuronal pentraxin-1",
  "term_id": "UNKNOWN:0003",
  "gene": "UniProtKB:Q15818"
}